collateral sprouting [GO:0048668] (biological process) Also known as: axon branching Relationships: is a type of GO:0048588; is a type of developmental growth involved in morphogenesis [GO:0060560]; is part of axonogenesis [GO:0007409] Subtypes: collateral sprouting in absence of injury [GO:0048669], collateral sprouting of intact axon in response to injury [GO:0048673], GO:0048674 Regulation: regulated by GO:0048670; negatively regulated by GO:0048671; positively regulated by positive regulation of collateral sprouting [GO:0048672] Sources: GOC:dgh, GOC:dph, GOC:jid, GOC:lm Definition: The process in which outgrowths develop from the shafts of existing axons.